{
  "gene_name": "Allergin-1",
  "gene_symbol": "MILR1",
  "term_label": "external side of plasma membrane",
  "term_id": "GO:0009897",
  "gene": "UniProtKB:Q7Z6M3"
}